{
  "gene_name": "Stereocilin",
  "term_label": "cell surface",
  "gene_symbol": "STRC",
  "term_id": "GO:0009986",
  "gene": "UniProtKB:Q7RTU9"
}